{
  "gene_symbol": "ADGRG6",
  "gene_name": "Adhesion G-protein coupled receptor G6",
  "term_label": "heart trabecula formation",
  "term_id": "GO:0060347",
  "gene": "UniProtKB:Q86SQ4"
}